{
  "gene_symbol": "CHRNA1",
  "term_label": "response to nicotine",
  "gene": "UniProtKB:P02708",
  "term_id": "GO:0035094",
  "gene_name": "Acetylcholine receptor subunit alpha"
}